{
  "term_id": "GO:0032588",
  "term_label": "trans-Golgi network membrane",
  "gene_name": "Secretory carrier-associated membrane protein 4",
  "gene_symbol": "SCAMP4",
  "gene": "UniProtKB:Q969E2"
}